{
  "term_label": "ATPase-coupled intramembrane lipid transporter activity",
  "term_id": "GO:0140326",
  "gene_name": "Phospholipid-transporting ATPase IK",
  "gene": "UniProtKB:O60423",
  "gene_symbol": "ATP8B3"
}